negative regulation of type II interferon production [GO:0032689] (biological process) Also known as: down regulation of interferon-gamma production, down-regulation of interferon-gamma production, downregulation of interferon-gamma production, negative regulation of interferon-gamma production, inhibition of interferon-gamma production, negative regulation of interferon-gamma biosynthetic process, negative regulation of interferon-gamma secretion References: PMID:15546383 Sources: GOC:add, GOC:mah Relationships: is a type of negative regulation of cytokine production [GO:0001818]; is a type of regulation of type II interferon production [GO:0032649]; negatively regulates type II interferon production [GO:0032609] Definition: Any process that stops, prevents, or reduces the frequency, rate, or extent of interferon-gamma production. Interferon-gamma is also known as type II interferon.